metaphase chromosome alignment [GO:0051310] (biological process) Sources: GOC:vw Also known as: chromosome congression Relationships: is_a chromosome localization [GO:0050000]; is part of nuclear chromosome segregation [GO:0098813] Definition: A chromosome localization process whereby chromosomes are positioned in a specific order and orientation at the metaphase plate (spindle equator), during chromosome segregation. This alignment ensures that each daughter cell will receive the correct number of chromosomes during cell division. Regulation: regulated by regulation of metaphase plate congression [GO:0090235] Subtypes: mitotic metaphase chromosome alignment [GO:0007080], meiotic metaphase chromosome alignment [GO:0051311]